hercynylcysteine sulfoxide lyase activity (ergothioneine-forming) [GO:1990411] (molecular function) Relationships: is a type of carbon-sulfur lyase activity [GO:0016846]; is part of ergothioneine biosynthetic process [GO:0052699] References: PMID:24828577 Definition: Catalysis of the reaction: hercynylcysteine sulfoxide + 2H+ = ergothioneine + pyruvate + ammonium.